TORC1 signaling [GO:0038202] (biological process) Relationships: is a type of TOR signaling [GO:0031929] Sources: GOC:lb Definition: A series of intracellular molecular signals mediated by TORC1; TOR (target of rapamycin) in complex with at least Raptor (regulatory-associated protein of TOR), or orthologs of, and other signaling components. Also known as: TORC1 signal transduction Regulation: regulated by regulation of TORC1 signaling [GO:1903432]; negatively regulated by negative regulation of TORC1 signaling [GO:1904262]; positively regulated by positive regulation of TORC1 signaling [GO:1904263]